carbon-oxygen lyase activity, acting on phosphates [GO:0016838] (molecular function) Sources: EC:4.2.3.- Definition: Catalysis of the cleavage of a carbon-oxygen bond by elimination of a phosphate. Relationships: is a type of carbon-oxygen lyase activity [GO:0016835] Subtypes: 3-dehydroquinate synthase activity [GO:0003856], 6-pyruvoyltetrahydropterin synthase activity [GO:0003874], chorismate synthase activity [GO:0004107], threonine synthase activity [GO:0004795], methylglyoxal synthase activity [GO:0008929], terpene synthase activity [GO:0010333], GO:0034004, S-linalool synthase activity [GO:0034007], R-linalool synthase activity [GO:0034008], ent-cassa-12,15-diene synthase activity [GO:0034277], stemar-13-ene synthase activity [GO:0034278], syn-pimara-7,15-diene synthase activity [GO:0034279], ent-sandaracopimaradiene synthase activity [GO:0034280], ent-pimara-8(14),15-diene synthase activity [GO:0034282], GO:0034283, phosphothreonine lyase activity [GO:0034598], (E)-beta-ocimene synthase activity [GO:0034768], aphidicolan-16 beta-ol synthase activity [GO:0046567], (-)-endo-fenchol synthase activity [GO:0050437], GO:0050459, sabinene-hydrate synthase activity [GO:0050469], taxadiene synthase activity [GO:0050553], abietadiene synthase activity [GO:0050554], ent-pimara-9(11),15-diene synthase activity [GO:0052674], levopimaradiene synthase activity [GO:0052678], GO:0052679, epi-isozizaene synthase activity [GO:0052680], GO:0052681, GO:0052682, GO:0052683, Labd-13(16),14-diene-9-ol synthase activity [GO:0062202], GO:0062203, GO:0062204, miltiradiene synthase activity [GO:0062205], manoyl oxide synthase activity [GO:0062206], (E,E)-geranyllinalool synthase activity [GO:0080013], endo-alpha-bergamotene synthase activity [GO:0102060], endo-beta-bergamotene synthase activity [GO:0102061], alpha-santalene synthase activity [GO:0102062], gamma-curcumene synthase activity [GO:0102064], (3R)-(E)-nerolidol synthase activity [GO:0102145], (+)-2-epi-prezizaene synthase activity [GO:0102201], sesquithujene synthase activity [GO:0102304], 1,8-cineole synthase activity [GO:0102313], GO:0102412, 5-epi-aristolochene synthase activity [GO:0102698], alpha-thujene synthase activity [GO:0102700], tricyclene synthase activity [GO:0102701], GO:0102702, camphene synthase activity [GO:0102703], alpha-copaene synthase activity [GO:0102877], GO:0102878, GO:0102879, (+)-beta-barbatene synthase activity [GO:0102881], beta-acoradiene synthase activity [GO:0102882], (+)-beta-chamigrene synthase activity [GO:0102883], GO:0102884, alpha-cuprenene synthase activity [GO:0102885], beta-sesquiphellandrene synthase activity [GO:0102887], beta-elemene synthase activity [GO:0102889], gamma-terpinene synthase activity [GO:0102903], germacrene C synthase activity [GO:0102904], valencene synthase activity [GO:0102905], GO:0102906, GO:0102931, 9,13-epoxylabda-14-ene synthase activity [GO:0106239], syn-isopimara-7,15-diene synthase activity [GO:0106243]